{
  "gene_symbol": "ZNF75A",
  "gene_name": "Zinc finger protein 75A",
  "term_id": "GO:0000977",
  "term_label": "RNA polymerase II transcription regulatory region sequence-specific DNA binding",
  "gene": "UniProtKB:Q96N20"
}